{
  "gene_symbol": "MAP3K11",
  "term_id": "GO:0007254",
  "term_label": "JNK cascade",
  "gene": "UniProtKB:Q16584",
  "gene_name": "Mitogen-activated protein kinase kinase kinase 11"
}